positive regulation of vesicle transport along microtubule [GO:1901610] (biological process) Relationships: is a type of positive regulation of intracellular transport [GO:0032388]; is a type of regulation of vesicle transport along microtubule [GO:1901608]; positively regulates vesicle transport along microtubule [GO:0047496] Subtypes: positive regulation of anterograde dense core granule transport [GO:1901953], positive regulation of retrograde dense core granule transport [GO:1901956], positive regulation of anterograde synaptic vesicle transport [GO:1903744] Also known as: activation of microtubule-based vesicle localization, positive regulation of microtubule-based vesicle localization, up regulation of microtubule-based vesicle localization, up regulation of vesicle transport along microtubule, up-regulation of microtubule-based vesicle localization, up-regulation of vesicle transport along microtubule, upregulation of microtubule-based vesicle localization, upregulation of vesicle transport along microtubule, activation of vesicle transport along microtubule Definition: Any process that activates or increases the frequency, rate or extent of vesicle transport along microtubule. Sources: GOC:TermGenie